{
  "term_id": "GO:0097500",
  "gene": "UniProtKB:Q3SXY8",
  "gene_name": "ADP-ribosylation factor-like protein 13B",
  "gene_symbol": "ARL13B",
  "term_label": "receptor localization to non-motile cilium"
}